interleukin-29 production [GO:0072631] (biological process) Note: Note that this term is in the subset of terms that should not be used for direct gene product annotation. Instead, select one of the 'regulation' children terms. Relationships: is a type of type III interferon production [GO:0034343] Definition: The appearance of interleukin-29 due to biosynthesis or secretion following a cellular stimulus, resulting in an increase in its intracellular or extracellular levels. Also known as: IL-29 production, IL29 production, interferon lambda 1 production, interleukin-29 secretion References: PMID:15546383 Sources: GOC:BHF, GOC:mah